absorption of UV light [GO:0016039] (biological process) Definition: The reception of a (UV light) photon by a cell, UV light being defined as having a wavelength within the range 13.6-400 nm. Relationships: is a type of GO:0016037 Sources: GOC:go_curators, ISBN:0198506732